{
  "term_label": "proteasome-activating activity",
  "gene": "UniProtKB:P43686",
  "gene_name": "26S proteasome regulatory subunit 6B",
  "gene_symbol": "PSMC4",
  "term_id": "GO:0036402"
}